{
  "gene_name": "T cell receptor alpha variable 36_delta variable 7",
  "term_id": "GO:0009617",
  "term_label": "response to bacterium",
  "gene_symbol": "TRAV36DV7",
  "gene": "UniProtKB:A0A075B6V5"
}